FAD transport [GO:0015883] (biological process) Definition: The directed movement of flavin-adenine dinucleotide (FAD) into, out of or within a cell, or between cells, by means of some agent such as a transporter or pore. FAD forms the coenzyme of the prosthetic group of various flavoprotein oxidoreductase enzymes, in which it functions as an electron acceptor by being reversibly converted to its reduced form. Sources: ISBN:0198506732 Also known as: flavin adenine dinucleotide transport, flavin-adenine dinucleotide transport Relationships: is a type of nucleotide transport [GO:0006862]; is a type of organic anion transport [GO:0015711] Subtypes: FAD transmembrane transport [GO:0035350]